{
  "gene_symbol": "ZNF587B",
  "term_label": "RNA polymerase II transcription regulatory region sequence-specific DNA binding",
  "gene": "UniProtKB:E7ETH6",
  "gene_name": "Zinc finger protein 587B",
  "term_id": "GO:0000977"
}